peripheral nervous system development [GO:0007422] (biological process) Sources: GOC:go_curators, UBERON:0000010 Definition: The process whose specific outcome is the progression of the peripheral nervous system over time, from its formation to the mature structure. The peripheral nervous system is one of the two major divisions of the nervous system. Nerves in the PNS connect the central nervous system (CNS) with sensory organs, other organs, muscles, blood vessels and glands. Relationships: is a type of system development [GO:0048731]; BFO_0000050 GO:0007399